chlorophyll fluorescence [GO:0090546] (biological process) Relationships: is a type of energy quenching [GO:1990066] Definition: The process by which excess light energy absorbed by chlorophyll and not used to drive photosynthesis is re-emitted as light. References: PMID:10938857